{
  "gene_symbol": "OR10X1",
  "gene_name": "Olfactory receptor 10X1",
  "term_label": "Unknown biological process",
  "term_id": "UNKNOWN:0002",
  "gene": "UniProtKB:Q8NGY0"
}